positive regulation of phospholipid scramblase activity [GO:1900163] (biological process) Relationships: is_a positive regulation of transporter activity [GO:0032411]; positively regulates phospholipid scramblase activity [GO:0017128] Definition: Any process that activates or increases the frequency, rate or extent of phospholipid scramblase activity. Also known as: up regulation of phospholipid scramblase activity, up-regulation of phospholipid scramblase activity, upregulation of phospholipid scramblase activity, activation of phospholipid scramblase activity Sources: GOC:TermGenie